ciliary transition fiber [GO:0097539] (cellular component) References: PMID:22653444, PMID:24231678, PMID:5064817, PMID:5335827 Sources: GOC:cilia, GOC:kmv, GOC:krc Also known as: transition fiber, transition fibre, cilial transition fiber, cilial transition fibre, ciliary transition fibre, cilium transition fiber, cilium transition fibre, centriolar distal appendage, distal appendage of basal body, distal appendage of centriole, distal appendage of mother centriole Definition: A nine-bladed, propeller-like protein complex that links the distal end of the basal body and the cilium to the plasma membrane. Functions in protein sorting and gating (i.e. active and passive transport of proteins in and out of the cilium). Relationships: is a type of GO:0140535; is part of cilium [GO:0005929] Note: In mammals, ciliary transition fibers comprise at least five components (Ccdc41/Cep83, Cep89/Cep123, Sclt1, Fbf1, and Cep164) (PMID:24469809).